{
  "gene": "UniProtKB:Q8IWS0",
  "term_label": "histone binding",
  "gene_name": "PHD finger protein 6",
  "gene_symbol": "PHF6",
  "term_id": "GO:0042393"
}